{
  "gene": "UniProtKB:Q32P44",
  "term_id": "GO:0000226",
  "term_label": "microtubule cytoskeleton organization",
  "gene_name": "Echinoderm microtubule-associated protein-like 3",
  "gene_symbol": "EML3"
}